nucleotide-excision repair, preincision complex assembly [GO:0006294] (biological process) References: PMID:10197977 Sources: GOC:elh Also known as: nucleotide-excision repair, preincision complex formation Definition: The aggregation, arrangement and bonding together of proteins on DNA to form the multiprotein complex involved in damage recognition, DNA helix unwinding, and endonucleolytic cleavage at the site of DNA damage. This assembly occurs before the phosphodiester backbone of the damaged strand is cleaved 3' and 5' of the site of DNA damage. Relationships: is a type of GO:0065004; is part of nucleotide-excision repair [GO:0006289]